{
  "gene_symbol": "TNFRSF17",
  "gene": "UniProtKB:Q02223",
  "term_id": "UNKNOWN:0003",
  "gene_name": "Tumor necrosis factor receptor superfamily member 17",
  "term_label": "Unknown cellular component"
}